discoidal high-density lipoprotein particle [GO:0034365] (cellular component) Definition: A newly formed high-density lipoprotein particle; consists of a phospholipid bilayer surrounded by two or more APOA1 molecules. The discoidal HDL particle is formed when lipid-free or lipid-poor APOA1 acquires phospholipids and unesterified cholesterol from either cell membranes or triglyceride-rich lipoproteins (undergoing lipolysis by lipoprotein lipase). Sources: GOC:BHF, GOC:expert_pt, GOC:mah, GOC:rl Also known as: discoidal HDL, nascent HDL, nascent high-density lipoprotein particle Relationships: is a type of high-density lipoprotein particle [GO:0034364]